{
  "term_label": "endoplasmic reticulum membrane",
  "term_id": "GO:0005789",
  "gene_name": "Calmegin",
  "gene_symbol": "CLGN",
  "gene": "UniProtKB:O14967"
}